{
  "gene_name": "Trem-like transcript 1 protein",
  "term_id": "GO:0007165",
  "gene_symbol": "TREML1",
  "gene": "UniProtKB:Q86YW5",
  "term_label": "signal transduction"
}